translation release factor complex [GO:0018444] (cellular component) Definition: A heterodimeric complex involved in the release of a nascent polypeptide chain from a ribosome. Also known as: peptide chain release factor, eukaryotic peptide chain release factor Relationships: is a type of protein-containing complex [GO:0032991]; is part of cytoplasm [GO:0005737] Sources: ISBN:0198547684